indole-3-acetyl-glycine synthetase activity [GO:0102047] (molecular function) Definition: Catalysis of the reaction: indole-3-acetate + glycine + ATP(4-) = H+ + indole-3-acetyl-glycine + AMP(2-) + diphosphoric acid. References: PMID:15659623 Sources: GOC:pz Relationships: is_a ligase activity, forming carbon-nitrogen bonds [GO:0016879]